{
  "term_label": "acetylcholine-gated monoatomic cation-selective channel activity",
  "gene_name": "Acetylcholine receptor subunit delta",
  "gene_symbol": "CHRND",
  "term_id": "GO:0022848",
  "gene": "UniProtKB:Q07001"
}